{
  "gene": "UniProtKB:Q7Z4H9",
  "term_id": "UNKNOWN:0001",
  "gene_symbol": "FAM220A",
  "gene_name": "Protein FAM220A",
  "term_label": "Unknown molecular function"
}